arachidonate 5-lipoxygenase activity [GO:0004051] (molecular function) Definition: Catalysis of the reaction: (5Z,8Z,11Z,14Z)-eicosatetraenoate + O2 = H2O + leukotriene A4. Sources: RHEA:32307 Also known as: leukotriene A4 synthase, LTA synthase activity, leukotriene-A(4) synthase activity, 5-delta-lipoxygenase activity, 5-lipoxygenase activity, 5Delta-lipoxygenase activity, C-5-lipoxygenase activity, arachidonate:oxygen 5-oxidoreductase activity, arachidonic 5-lipoxygenase activity, arachidonic acid 5-lipoxygenase activity, delta(5)-lipoxygenase activity, delta5-lipoxygenase activity, leukotriene-A4 synthase activity Note: Note that this is a multi-step reaction. Relationships: is a type of GO:0016702